{
  "term_label": "centrosome",
  "gene": "UniProtKB:Q96ED9",
  "gene_name": "Protein Hook homolog 2",
  "gene_symbol": "HOOK2",
  "term_id": "GO:0005813"
}